N,N-dimethylaniline monooxygenase activity [GO:0004499] (molecular function) Relationships: is a type of oxidoreductase activity, acting on paired donors, with incorporation or reduction of molecular oxygen, NAD(P)H as one donor, and incorporation of one atom of oxygen [GO:0016709] Also known as: flavin-containing monooxygenase activity, dimethylaniline monooxygenase (N-oxide-forming) activity, methylphenyltetrahydropyridine N-monooxygenase activity, 1-methyl-4-phenyl-1,2,3,6-tetrahydropyridine:oxygen N-oxidoreductase activity, DMA oxidase activity, FAD-containing monooxygenase activity, FMO activity, N,N-dimethylaniline,NADPH:oxygen oxidoreductase (N-oxide-forming), Ziegler's enzyme, dimethylaniline N-oxidase activity, dimethylaniline oxidase activity, flavin mixed function oxidase activity, flavin monooxygenase activity, mixed-function amine oxidase activity Sources: RHEA:24468 Definition: Catalysis of the reaction: N,N-dimethylaniline + NADPH + H+ + O2 = N,N-dimethylaniline N-oxide + NADP+ + H2O.